maintenance of neuroblast polarity [GO:0045201] (biological process) Definition: The maintenance of the apicobasal polarity of a neuroblast cell, a progenitor of the central nervous system. Also known as: maintenance of neuroblast cell polarity Relationships: is a type of GO:0030011; is a type of establishment or maintenance of neuroblast polarity [GO:0045196] Sources: GOC:bf, GOC:mtg_sensu